single-species biofilm formation in or on host organism [GO:0044407] (biological process) Sources: GOC:cc Definition: A process in which microorganisms of the same species attach to and grow in or on a host species, and produce extracellular polymers that facilitate attachment and matrix formation, resulting in a change in the microorganisms' growth rate and gene transcription. The host is defined as the larger of the organisms involved in a symbiotic interaction. Relationships: is a type of single-species biofilm formation [GO:0044010]; is a type of GO:0044406 Regulation: regulated by regulation of single-species biofilm formation in or on host organism [GO:1900228]; negatively regulated by negative regulation of single-species biofilm formation in or on host organism [GO:1900229]; RO_0002213 by GO:1900230